{
  "gene": "UniProtKB:Q08752",
  "gene_symbol": "PPID",
  "gene_name": "Peptidyl-prolyl cis-trans isomerase D",
  "term_label": "protein folding",
  "term_id": "GO:0006457"
}